tertiary granule lumen [GO:1904724] (cellular component) Also known as: membrane-enclosed lumen of gelatinase granule, membrane-enclosed lumen of tertiary granule, tertiary granule membrane-enclosed lumen, gelatinase granule membrane-enclosed lumen References: PMID:23650620 Sources: GOC:TermGenie, GO_REF:0000064 Definition: Any membrane-enclosed lumen that is part of a tertiary granule. Relationships: is a type of intracellular organelle lumen [GO:0070013]; is part of tertiary granule [GO:0070820]